{
  "term_label": "zinc ion binding",
  "gene": "UniProtKB:P00325",
  "gene_symbol": "ADH1B",
  "term_id": "GO:0008270",
  "gene_name": "All-trans-retinol dehydrogenase [NAD(+)] ADH1B"
}